exon-exon junction subcomplex mago-y14 [GO:1990501] (cellular component) Also known as: MGN-RBM8A complex, exon junction subcomplex MAGOH-Y14, mago-y14 complex Relationships: is a type of exon-exon junction complex [GO:0035145]; is_a GO:1903503 References: PMID:12730685 Sources: GOC:bhm Note: An example of this is Mago in drome (P49028) in PMID:12730685 (inferred from direct assay). Definition: Component of the core exon-exon-junction complex (EJC). Fairly conserved in eukaryotes; in Drosophila, consists of the Mago and Y14 (tsunagi) gene products. Important for coupling nuclear and cytoplasmic events in gene expression. Inhibits the ATPase activity of eIF4AIII (Q9VHS8) to ensure a stable association of the EJC core with the mRNA.